vacuole [GO:0005773] (CC) Relationships: is_a intracellular membrane-bounded organelle [GO:0043231]; is part of GO:0005737 Subtypes: GO:0000322, lytic vacuole [GO:0000323], plant-type vacuole [GO:0000325], contractile vacuole [GO:0000331], autophagosome [GO:0005776], GO:0032195 Sources: GOC:mtg_sensu, ISBN:0198506732 Definition: A closed structure, found only in eukaryotic cells, that is completely surrounded by unit membrane and contains liquid material. Cells contain one or several vacuoles, that may have different functions from each other. Vacuoles have a diverse array of functions. They can act as a storage organelle for nutrients or waste products, as a degradative compartment, as a cost-effective way of increasing cell size, and as a homeostatic regulator controlling both turgor pressure and pH of the cytosol. Also known as: vacuolar carboxypeptidase Y